{
  "gene_symbol": "RAB31",
  "term_label": "Golgi to plasma membrane protein transport",
  "gene_name": "Ras-related protein Rab-31",
  "term_id": "GO:0043001",
  "gene": "UniProtKB:Q13636"
}